{
  "term_id": "UNKNOWN:0001",
  "gene_symbol": "CST6",
  "term_label": "Unknown molecular function",
  "gene": "UniProtKB:Q15828",
  "gene_name": "Cystatin-M"
}